{
  "term_id": "GO:0006357",
  "gene_symbol": "ZNF699",
  "gene_name": "Zinc finger protein 699",
  "gene": "UniProtKB:Q32M78",
  "term_label": "regulation of transcription by RNA polymerase II"
}